negative regulation of macropinocytosis [GO:1905302] (biological process) Relationships: is a type of negative regulation of pinocytosis [GO:0048550]; is a type of regulation of macropinocytosis [GO:1905301]; negatively regulates macropinocytosis [GO:0044351] Definition: Any process that stops, prevents or reduces the frequency, rate or extent of macropinocytosis. References: PMID:18691641 Sources: GOC:PARL, GOC:TermGenie, GOC:pad, GO_REF:0000058 Also known as: down regulation of macropinocytosis, down-regulation of macropinocytosis, downregulation of macropinocytosis, inhibition of macropinocytosis